TBP-class protein binding [GO:0017025] (molecular function) Relationships: is a type of GO:0140296 Definition: Binding to a member of the class of TATA-binding proteins (TBP), including any of the TBP-related factors (TRFs). Also known as: TATA-binding protein binding, TBP binding, TBP-related factor (TRF) protein binding References: PMID:1509519, PMID:16858867 Sources: GOC:jl, GOC:txnOH